positive regulation of monoatomic ion transport [GO:0043270] (biological process) Definition: Any process that activates or increases the frequency, rate or extent of the directed movement of charged atoms or small charged molecules into, out of or within a cell, or between cells, by means of some agent such as a transporter or pore. Sources: GOC:jl Relationships: is a type of regulation of monoatomic ion transport [GO:0043269]; is_a positive regulation of transport [GO:0051050]; positively regulates monoatomic ion transport [GO:0006811] Subtypes: positive regulation of sodium ion transport [GO:0010765], positive regulation of serotonin secretion [GO:0014064], positive regulation of iron ion transport [GO:0034758], positive regulation of monoatomic ion transmembrane transport [GO:0034767], positive regulation of potassium ion transport [GO:0043268], positive regulation of calcium ion transport [GO:0051928], positive regulation of monoatomic anion transport [GO:1903793] Also known as: up regulation of ion transport, up-regulation of ion transport, upregulation of ion transport, activation of ion transport, stimulation of ion transport